{
  "gene_symbol": "LTV1",
  "gene": "UniProtKB:Q96GA3",
  "gene_name": "Protein LTV1 homolog",
  "term_id": "GO:0042274",
  "term_label": "ribosomal small subunit biogenesis"
}